{
  "gene": "UniProtKB:Q9NTJ3",
  "term_label": "meiotic chromosome segregation",
  "term_id": "GO:0045132",
  "gene_symbol": "SMC4",
  "gene_name": "Structural maintenance of chromosomes protein 4"
}